{
  "gene_symbol": "PTPRR",
  "term_label": "cell junction",
  "gene_name": "Receptor-type tyrosine-protein phosphatase R",
  "term_id": "GO:0030054",
  "gene": "UniProtKB:Q15256"
}